cellular response to estradiol stimulus [GO:0071392] (biological process) Sources: GOC:mah Relationships: is a type of response to estradiol [GO:0032355]; is a type of cellular response to lipid [GO:0071396]; is a type of cellular response to oxygen-containing compound [GO:1901701] Definition: Any process that results in a change in state or activity of a cell (in terms of movement, secretion, enzyme production, gene expression, etc.) as a result of stimulus by estradiol, a C18 steroid hormone hydroxylated at C3 and C17 that acts as a potent estrogen. Also known as: cellular response to E2 stimulus